{
  "gene_name": "Integral membrane protein GPR137",
  "gene": "UniProtKB:Q96N19",
  "term_id": "GO:0005765",
  "gene_symbol": "GPR137",
  "term_label": "lysosomal membrane"
}